{
  "term_label": "nuclear periphery",
  "gene_name": "LEM domain-containing protein 2",
  "gene_symbol": "LEMD2",
  "gene": "UniProtKB:Q8NC56",
  "term_id": "GO:0034399"
}